{
  "term_id": "GO:0001580",
  "gene": "UniProtKB:Q9NYV7",
  "gene_name": "Taste receptor type 2 member 16",
  "term_label": "detection of chemical stimulus involved in sensory perception of bitter taste",
  "gene_symbol": "TAS2R16"
}